{
  "term_id": "GO:0002223",
  "gene_name": "Natural killer cells antigen CD94",
  "gene": "UniProtKB:Q13241",
  "term_label": "stimulatory C-type lectin receptor signaling pathway",
  "gene_symbol": "KLRD1"
}